negative regulation of vasculogenesis [GO:2001213] (biological process) Sources: GOC:obol Also known as: negative regulation of vascular morphogenesis Relationships: is a type of GO:0045596; is a type of regulation of vasculogenesis [GO:2001212]; negatively regulates vasculogenesis [GO:0001570] Definition: Any process that stops, prevents or reduces the frequency, rate or extent of vasculogenesis.